transcription factor TFIIA complex [GO:0005672] (cellular component) Relationships: is a type of RNA polymerase II transcription regulator complex [GO:0090575]; is part of RNA polymerase II, holoenzyme [GO:0016591] Definition: A component of the transcription machinery of RNA Polymerase II. In humans, TFIIA is a heterotrimer composed of an alpha (P35), beta (P19) and gamma subunits (P12). References: PMID:17560669 Sources: GOC:jl